{
  "gene_name": "Myosin regulatory light chain 2, ventricular_cardiac muscle isoform",
  "term_id": "GO:0005737",
  "gene_symbol": "MYL2",
  "term_label": "cytoplasm",
  "gene": "UniProtKB:P10916"
}